{
  "gene_name": "Zinc finger protein 497",
  "gene": "UniProtKB:Q6ZNH5",
  "term_label": "regulation of transcription by RNA polymerase II",
  "gene_symbol": "ZNF497",
  "term_id": "GO:0006357"
}